alpha-ketoglutarate transport [GO:0015742] (biological process) Sources: GOC:krc Relationships: is a type of dicarboxylic acid transport [GO:0006835] Also known as: 2-oxoglutarate transport, mitochondrial alpha-ketoglutarate/malate transport Subtypes: mitochondrial alpha-ketoglutarate transmembrane transport [GO:1990550] Definition: The directed movement of alpha-ketoglutarate into, out of or within a cell, or between cells, by means of some agent such as a transporter or pore.